{
  "gene_name": "Origin recognition complex subunit 3",
  "term_id": "GO:0003688",
  "gene_symbol": "ORC3",
  "term_label": "DNA replication origin binding",
  "gene": "UniProtKB:Q9UBD5"
}